regulation of action potential firing rate [GO:0099605] (biological process) Sources: ISBN:978-0071390118 Definition: Any process that regulates the frequency of action potentials in a spike train. Relationships: is a type of regulation of action potential [GO:0098900]